{
  "gene_symbol": "CD80",
  "term_id": "GO:0042130",
  "gene_name": "T-lymphocyte activation antigen CD80",
  "gene": "UniProtKB:P33681",
  "term_label": "negative regulation of T cell proliferation"
}